{
  "term_label": "ribonucleoside-diphosphate reductase activity, thioredoxin disulfide as acceptor",
  "gene_symbol": "RRM1",
  "gene_name": "Ribonucleoside-diphosphate reductase large subunit",
  "gene": "UniProtKB:P23921",
  "term_id": "GO:0004748"
}